{
  "gene_name": "Kelch-like protein 29",
  "term_label": "cytoplasm",
  "gene": "UniProtKB:Q96CT2",
  "gene_symbol": "KLHL29",
  "term_id": "GO:0005737"
}